negative regulation of miRNA catabolic process [GO:2000626] (biological process) Definition: Any process that stops, prevents or reduces the frequency, rate or extent of miRNA catabolic process. Sources: GOC:dph Relationships: is a type of GO:1902369; is a type of regulation of miRNA catabolic process [GO:2000625]; is a type of negative regulation of miRNA metabolic process [GO:2000629]; negatively regulates miRNA catabolic process [GO:0010587] Also known as: negative regulation of microRNA catabolic process